positive regulation of juvenile hormone catabolic process [GO:0045971] (biological process) Relationships: is a type of positive regulation of hormone metabolic process [GO:0032352]; is a type of regulation of juvenile hormone catabolic process [GO:0045952]; is a type of positive regulation of lipid catabolic process [GO:0050996]; RO_0002213 juvenile hormone catabolic process [GO:0006719] Sources: GOC:go_curators Also known as: positive regulation of juvenile hormone breakdown, positive regulation of juvenile hormone catabolism, positive regulation of juvenile hormone degradation, up regulation of juvenile hormone catabolic process, up-regulation of juvenile hormone catabolic process, upregulation of juvenile hormone catabolic process, activation of juvenile hormone catabolic process, stimulation of juvenile hormone catabolic process Definition: Any process that activates or increases the frequency, rate or extent of the chemical reactions and pathways resulting in the breakdown of juvenile hormone.